{
  "term_label": "ferrous iron binding",
  "term_id": "GO:0008198",
  "gene": "UniProtKB:Q8N4E7",
  "gene_symbol": "FTMT",
  "gene_name": "Ferritin, mitochondrial"
}